{
  "term_id": "GO:0000981",
  "gene": "UniProtKB:Q9UD57",
  "gene_name": "NK1 transcription factor-related protein 2",
  "term_label": "DNA-binding transcription factor activity, RNA polymerase II-specific",
  "gene_symbol": "NKX1-2"
}